positive regulation of 17-methylnonadec-1-ene biosynthetic process [GO:1900958] (biological process) Sources: GOC:TermGenie, GOC:mengo_curators Relationships: is a type of GO:1900913; is a type of GO:1900956; positively regulates 17-methylnonadec-1-ene biosynthetic process [GO:1900883] Definition: Any process that activates or increases the frequency, rate or extent of 17-methylnonadec-1-ene biosynthetic process. Also known as: activation of 17-methylnonadec-1-ene anabolism, activation of 17-methylnonadec-1-ene biosynthesis, activation of 17-methylnonadec-1-ene formation, activation of 17-methylnonadec-1-ene synthesis, positive regulation of 17-methylnonadec-1-ene anabolism, positive regulation of 17-methylnonadec-1-ene biosynthesis, positive regulation of 17-methylnonadec-1-ene formation, positive regulation of 17-methylnonadec-1-ene synthesis, up regulation of 17-methylnonadec-1-ene anabolism, up regulation of 17-methylnonadec-1-ene biosynthesis, up regulation of 17-methylnonadec-1-ene biosynthetic process, up regulation of 17-methylnonadec-1-ene formation, up regulation of 17-methylnonadec-1-ene synthesis, up-regulation of 17-methylnonadec-1-ene anabolism, up-regulation of 17-methylnonadec-1-ene biosynthesis, up-regulation of 17-methylnonadec-1-ene biosynthetic process, up-regulation of 17-methylnonadec-1-ene formation, up-regulation of 17-methylnonadec-1-ene synthesis, upregulation of 17-methylnonadec-1-ene anabolism, upregulation of 17-methylnonadec-1-ene biosynthesis, upregulation of 17-methylnonadec-1-ene biosynthetic process, upregulation of 17-methylnonadec-1-ene formation, upregulation of 17-methylnonadec-1-ene synthesis, activation of 17-methylnonadec-1-ene biosynthetic process